{
  "gene": "UniProtKB:Q96AJ9",
  "gene_name": "Vesicle transport through interaction with t-SNAREs homolog 1A",
  "gene_symbol": "VTI1A",
  "term_label": "Golgi apparatus",
  "term_id": "GO:0005794"
}